{
  "term_id": "UNKNOWN:0002",
  "term_label": "Unknown biological process",
  "gene_name": "Zinc finger SWIM domain-containing protein 6",
  "gene_symbol": "ZSWIM6",
  "gene": "UniProtKB:Q9HCJ5"
}